{
  "gene_name": "Cylicin-1",
  "gene": "UniProtKB:P35663",
  "gene_symbol": "CYLC1",
  "term_label": "Unknown molecular function",
  "term_id": "UNKNOWN:0001"
}